{
  "gene_symbol": "HIVEP1",
  "term_id": "GO:0000981",
  "gene": "UniProtKB:P15822",
  "term_label": "DNA-binding transcription factor activity, RNA polymerase II-specific",
  "gene_name": "Zinc finger protein 40"
}